protein neddylation [GO:0045116] (biological process) Note: Note that currently, the only known substrates of neddylation are cullin family proteins. Regulation: regulated by GO:2000434; RO_0002212 by negative regulation of protein neddylation [GO:2000435]; positively regulated by positive regulation of protein neddylation [GO:2000436] References: PMID:11698580 Definition: Covalent attachment of the ubiquitin-like protein NEDD8 (RUB1) to another protein. Also known as: RUB1-protein conjugation Relationships: is_a protein modification by small protein conjugation [GO:0032446]